{
  "gene_symbol": "GFI1",
  "term_id": "GO:0003700",
  "gene_name": "Zinc finger protein Gfi-1",
  "gene": "UniProtKB:Q99684",
  "term_label": "DNA-binding transcription factor activity"
}